{
  "term_label": "negative regulation of dendritic cell differentiation",
  "gene_name": "Transmembrane protein 176B",
  "term_id": "GO:2001199",
  "gene_symbol": "TMEM176B",
  "gene": "UniProtKB:Q3YBM2"
}